{
  "gene_name": "Claudin-2",
  "term_label": "bicellular tight junction",
  "term_id": "GO:0005923",
  "gene": "UniProtKB:P57739",
  "gene_symbol": "CLDN2"
}